{
  "gene": "UniProtKB:Q86VI4",
  "gene_name": "Lysosomal-associated transmembrane protein 4B",
  "term_id": "GO:0005765",
  "gene_symbol": "LAPTM4B",
  "term_label": "lysosomal membrane"
}